{
  "term_id": "GO:0031012",
  "gene": "UniProtKB:Q14055",
  "gene_name": "Collagen alpha-2(IX) chain",
  "term_label": "extracellular matrix",
  "gene_symbol": "COL9A2"
}